{
  "gene": "UniProtKB:Q9BQ16",
  "term_id": "GO:0005615",
  "gene_name": "Testican-3",
  "gene_symbol": "SPOCK3",
  "term_label": "extracellular space"
}